{
  "gene": "UniProtKB:P43080",
  "gene_name": "Guanylyl cyclase-activating protein 1",
  "term_label": "visual perception",
  "gene_symbol": "GUCA1A",
  "term_id": "GO:0007601"
}